{
  "gene": "UniProtKB:A0A0B4J266",
  "term_id": "UNKNOWN:0002",
  "gene_name": "T cell receptor alpha variable 41",
  "gene_symbol": "TRAV41",
  "term_label": "Unknown biological process"
}